negative regulation of hydrogen peroxide-mediated programmed cell death [GO:1901299] (biological process) Relationships: is a type of negative regulation of programmed cell death [GO:0043069]; is a type of GO:1901298; negatively regulates GO:0010421 Also known as: down regulation of hydrogen peroxide-mediated programmed cell death, down-regulation of hydrogen peroxide-mediated programmed cell death, downregulation of hydrogen peroxide-mediated programmed cell death, inhibition of hydrogen peroxide-mediated programmed cell death Definition: Any process that stops, prevents or reduces the frequency, rate or extent of hydrogen peroxide-mediated programmed cell death. Subtypes: GO:1903751 Sources: GOC:BHF, GOC:TermGenie